methane monooxygenase complex [GO:0015050] (cellular component) Definition: A protein complex that possesses methane monooxygenase activity; dimeric and trimeric complexes have been characterized. References: PMID:15544 Sources: GOC:mah Relationships: is a type of GO:1990204